{
  "gene_symbol": "HRH4",
  "gene_name": "Histamine H4 receptor",
  "term_id": "GO:0004969",
  "term_label": "histamine receptor activity",
  "gene": "UniProtKB:Q9H3N8"
}